{
  "gene_symbol": "PMF1",
  "gene_name": "Polyamine-modulated factor 1",
  "gene": "UniProtKB:Q6P1K2",
  "term_label": "Unknown molecular function",
  "term_id": "UNKNOWN:0001"
}